{
  "term_id": "UNKNOWN:0002",
  "term_label": "Unknown biological process",
  "gene_symbol": "OGFOD3",
  "gene": "UniProtKB:Q6PK18",
  "gene_name": "2-oxoglutarate and iron-dependent oxygenase domain-containing protein 3"
}